{
  "term_label": "transmembrane signaling receptor activity",
  "term_id": "GO:0004888",
  "gene_symbol": "SORCS2",
  "gene_name": "VPS10 domain-containing receptor SorCS2",
  "gene": "UniProtKB:Q96PQ0"
}